{
  "gene_symbol": "O00370",
  "term_id": "UNKNOWN:0003",
  "gene": "UniProtKB:O00370",
  "gene_name": "LINE-1 retrotransposable element ORF2 protein",
  "term_label": "Unknown cellular component"
}